{
  "gene_symbol": "HEATR3",
  "gene": "UniProtKB:Q7Z4Q2",
  "term_id": "GO:0006606",
  "gene_name": "HEAT repeat-containing protein 3",
  "term_label": "protein import into nucleus"
}